{
  "gene_symbol": "ZFAND1",
  "term_label": "Unknown molecular function",
  "gene_name": "AN1-type zinc finger protein 1",
  "gene": "UniProtKB:Q8TCF1",
  "term_id": "UNKNOWN:0001"
}